positive regulation of CD40 signaling pathway [GO:2000350] (biological process) Also known as: positive regulation of CD40 signalling pathway Relationships: is a type of positive regulation of signal transduction [GO:0009967]; is a type of regulation of CD40 signaling pathway [GO:2000348]; positively regulates CD40 signaling pathway [GO:0023035] Definition: Any process that activates or increases the frequency, rate or extent of signaling via the CD40 signaling pathway. Sources: GOC:BHF, GOC:mah